negative regulation of microglial cell migration [GO:1904140] (biological process) Definition: Any process that stops, prevents or reduces the frequency, rate or extent of microglial cell migration. References: PMID:19100238 Sources: GOC:BHF, GOC:TermGenie, GOC:nc, GO_REF:0000058 Also known as: down regulation of microglial cell migration, down-regulation of microglial cell migration, downregulation of microglial cell migration, inhibition of microglial cell migration Relationships: is a type of negative regulation of glial cell migration [GO:1903976]; is a type of regulation of microglial cell migration [GO:1904139]; is a type of negative regulation of macrophage migration [GO:1905522]; negatively regulates microglial cell migration [GO:1904124]